4alpha-hydroxymethyl,4beta,14alpha-dimethyl-9beta,19-cyclo-5alpha-ergost-24(241)-en-3beta-ol-4alpha-methyl oxidase activity [GO:0102172] (molecular function) Relationships: is a type of oxidoreductase activity, acting on paired donors, with incorporation or reduction of molecular oxygen, NAD(P)H as one donor, and incorporation of one atom of oxygen [GO:0016709] Definition: Catalysis of the reaction: 4alpha-hydroxymethyl,4beta,14alpha-dimethyl-9beta,19-cyclo-5alpha-ergost-24(241)-en-3beta-ol + NADH + O2 + H+ = 4alpha-formyl,4beta,14alpha-dimethyl-9beta,19-cyclo-5alpha-ergost-24(241)-en-3beta-ol + NAD + 2 H2O. Sources: GOC:pz, RHEA:58860